{
  "term_label": "regulation of mitotic metaphase/anaphase transition",
  "gene": "UniProtKB:O00762",
  "gene_symbol": "UBE2C",
  "gene_name": "Ubiquitin-conjugating enzyme E2 C",
  "term_id": "GO:0030071"
}